{
  "term_id": "GO:0031410",
  "gene": "UniProtKB:P49757",
  "term_label": "cytoplasmic vesicle",
  "gene_symbol": "NUMB",
  "gene_name": "Protein numb homolog"
}